oxaloacetate tautomerase activity [GO:0050163] (molecular function) Definition: Catalysis of the reaction: oxaloacetate = <stereo>enol</stereo>-oxaloacetate. Relationships: is a type of intramolecular oxidoreductase activity, interconverting keto- and enol-groups [GO:0016862] Also known as: oxalacetic keto-enol isomerase activity, oxaloacetate keto-enol tautomerase activity, oxaloacetate keto-enol-isomerase activity Sources: EC:5.3.2.2, RHEA:16021